{
  "gene_name": "Epidermal growth factor receptor substrate 15",
  "term_label": "clathrin coat of coated pit",
  "gene_symbol": "EPS15",
  "gene": "UniProtKB:P42566",
  "term_id": "GO:0030132"
}